{
  "gene": "UniProtKB:Q9H814",
  "gene_symbol": "PHAX",
  "gene_name": "Phosphorylated adapter RNA export protein",
  "term_id": "GO:0005634",
  "term_label": "nucleus"
}